homoserine transport [GO:0042968] (biological process) Relationships: is a type of GO:0015804; is a type of carboxylic acid transport [GO:0046942]; is a type of GO:0071705 Definition: The directed movement of homoserine, alpha-amino-gamma-hydroxybutyric acid, an intermediate in the biosynthesis of cystathionine, threonine and methionine, into, out of or within a cell, or between cells, by means of some agent such as a transporter or pore. Sources: GOC:go_curators, ISBN:0198506732